{
  "term_label": "cytosol",
  "gene_name": "Retrotransposon-derived protein PEG10",
  "gene": "UniProtKB:Q86TG7",
  "term_id": "GO:0005829",
  "gene_symbol": "PEG10"
}